mononuclear cell proliferation [GO:0032943] (biological process) Sources: GOC:add Relationships: is a type of GO:0070661 Definition: The expansion of a mononuclear cell population by cell division. A mononuclear cell is a leukocyte with a single non-segmented nucleus in the mature form. Regulation: regulated by regulation of mononuclear cell proliferation [GO:0032944]; negatively regulated by negative regulation of mononuclear cell proliferation [GO:0032945]; positively regulated by positive regulation of mononuclear cell proliferation [GO:0032946] Also known as: PBMC proliferation, peripheral blood mononuclear cell proliferation Subtypes: dendritic cell proliferation [GO:0044565], GO:0046651